{
  "term_label": "acyl-CoA dehydrogenase activity",
  "term_id": "GO:0003995",
  "gene_symbol": "ACAD10",
  "gene": "UniProtKB:Q6JQN1",
  "gene_name": "Acyl-CoA dehydrogenase family member 10"
}